{
  "gene_symbol": "TAAR3P",
  "term_label": "plasma membrane",
  "gene_name": "Putative trace amine-associated receptor 3",
  "gene": "UniProtKB:Q9P1P4",
  "term_id": "GO:0005886"
}